{
  "gene": "UniProtKB:P50226",
  "gene_name": "Sulfotransferase 1A2",
  "term_label": "aryl sulfotransferase activity",
  "gene_symbol": "SULT1A2",
  "term_id": "GO:0004062"
}